epoxyqueuosine reductase activity [GO:0052693] (MF) References: PMID:21502530 Sources: RHEA:32159 Relationships: is a type of oxidoreductase activity, acting on CH or CH2 groups [GO:0016725] Definition: Catalysis of the reaction: epoxyqueuosine in tRNA + reductant = queuosine in tRNA + oxidised reductant.